{
  "gene": "UniProtKB:Q9BVC4",
  "term_label": "regulation of actin cytoskeleton organization",
  "term_id": "GO:0032956",
  "gene_name": "Target of rapamycin complex subunit LST8",
  "gene_symbol": "MLST8"
}